neosartoricin catabolic process [GO:1902049] (biological process) References: PMID:23368997 Sources: GOC:TermGenie, GOC:di Also known as: neosartoricin breakdown, neosartoricin catabolism, neosartoricin degradation Relationships: is a type of phenol-containing compound catabolic process [GO:0019336]; is a type of polyketide catabolic process [GO:0030640]; is_a ketone catabolic process [GO:0042182]; is a type of GO:0046164; is a type of GO:1902644 Definition: The chemical reactions and pathways resulting in the breakdown of neosartoricin.